fibroblast growth factor receptor signaling pathway involved in heart development [GO:0061313] (BP) Sources: GOC:mtg_heart Also known as: fibroblast growth factor receptor signalling pathway involved in heart development Definition: The series of molecular signals generated as a consequence of a fibroblast growth factor receptor binding to one of its physiological ligands and contributing to the progression of the heart over time. Relationships: is a type of fibroblast growth factor receptor signaling pathway [GO:0008543]; is_a cell surface receptor signaling pathway involved in heart development [GO:0061311]